{
  "term_label": "Unknown cellular component",
  "term_id": "UNKNOWN:0003",
  "gene": "UniProtKB:Q9Y2K6",
  "gene_name": "Ubiquitin carboxyl-terminal hydrolase 20",
  "gene_symbol": "USP20"
}